dopamine binding [GO:0035240] (molecular function) Definition: Binding to dopamine, a catecholamine neurotransmitter formed by aromatic-L-amino-acid decarboxylase from 3,4-dihydroxy-L-phenylalanine. Sources: ISBN:0198506732 Relationships: is a type of cation binding [GO:0043169]; is a type of catecholamine binding [GO:1901338]